{
  "term_id": "GO:0015440",
  "term_label": "ABC-type peptide transporter activity",
  "gene_name": "Antigen peptide transporter 2",
  "gene_symbol": "TAP2",
  "gene": "UniProtKB:Q03519"
}